{
  "term_label": "phosphatidylethanolamine binding",
  "gene_symbol": "MAP1LC3B2",
  "gene": "UniProtKB:A6NCE7",
  "gene_name": "Microtubule-associated proteins 1A_1B light chain 3 beta 2",
  "term_id": "GO:0008429"
}